positive regulation of calcium ion transmembrane transport via high voltage-gated calcium channel [GO:1904879] (biological process) Relationships: is a type of regulation of calcium ion transmembrane transport via high voltage-gated calcium channel [GO:1902514]; is a type of positive regulation of calcium ion transmembrane transport [GO:1904427]; positively regulates calcium ion transmembrane transport via high voltage-gated calcium channel [GO:0061577] Also known as: up regulation of generation of L-type calcium current, up-regulation of generation of L-type calcium current, upregulation of generation of L-type calcium current, activation of generation of L-type calcium current, positive regulation of generation of L-type calcium current References: PMID:23071515 Sources: GOC:TermGenie, GO_REF:0000058 Definition: Any process that activates or increases the frequency, rate or extent of calcium ion transmembrane transport via high voltage-gated calcium channel.